{
  "gene_name": "Protein kinase C theta type",
  "term_id": "GO:0035556",
  "gene": "UniProtKB:Q04759",
  "gene_symbol": "PRKCQ",
  "term_label": "intracellular signal transduction"
}